pericyte cell differentiation [GO:1904238] (biological process) Definition: The process in which a relatively unspecialized cell acquires the specialized features of a pericyte cell. References: PMID:23868830 Sources: GOC:TermGenie, GOC:dph, GO_REF:0000086 Relationships: is a type of cell differentiation [GO:0030154] Subtypes: mesangial cell differentiation [GO:0072007]